temperature-gated cation channel activity [GO:0097604] (molecular function) Definition: Enables the transmembrane transfer of a cation by a channel that opens in response to a temperature stimulus (e.g. exposure to a temperature range different than the optimal temperature for that organism). References: PMID:23027824 Sources: GOC:ha, GOC:pr Relationships: is a type of monoatomic cation channel activity [GO:0005261]; is_a temperature-gated ion channel activity [GO:0097603] Also known as: temperature gated cation channel activity, temperature-activated cation channel activity, temperature-dependent cation channel activity, heat-activated cation channel activity